glycolytic process from mannose through fructose-6-phosphate [GO:0061619] (biological process) Definition: The chemical reactions and pathways resulting in the breakdown of mannose into pyruvate, occurring through a fructose-6-phosphate intermediate, with the concomitant production of ATP and NADH. Sources: GOC:dph, ISBN:0201090910, ISBN:0879010479 Relationships: is a type of mannose catabolic process [GO:0019309]; is_a glycolytic process through fructose-6-phosphate [GO:0061615]; has part mannose to fructose-6-phosphate catabolic process [GO:0061611]